{
  "gene_name": "Proteinase-activated receptor 2",
  "gene": "UniProtKB:P55085",
  "term_id": "GO:0070374",
  "term_label": "positive regulation of ERK1 and ERK2 cascade",
  "gene_symbol": "F2RL1"
}